{
  "term_label": "cytoplasm",
  "gene_name": "Tubulin beta-6 chain",
  "gene": "UniProtKB:Q9BUF5",
  "term_id": "GO:0005737",
  "gene_symbol": "TUBB6"
}